{
  "gene_name": "Multiple epidermal growth factor-like domains protein 6",
  "gene_symbol": "MEGF6",
  "gene": "UniProtKB:O75095",
  "term_id": "GO:0005886",
  "term_label": "plasma membrane"
}